{
  "term_label": "odorant binding",
  "gene_symbol": "OR10J1",
  "term_id": "GO:0005549",
  "gene_name": "Olfactory receptor 10J1",
  "gene": "UniProtKB:P30954"
}